{
  "gene": "UniProtKB:Q69YN2",
  "gene_name": "CWF19-like protein 1",
  "term_id": "GO:0071014",
  "gene_symbol": "CWF19L1",
  "term_label": "post-mRNA release spliceosomal complex"
}